{
  "gene_name": "DNA-directed RNA polymerases I and III subunit RPAC1",
  "gene": "UniProtKB:O15160",
  "term_id": "UNKNOWN:0002",
  "term_label": "Unknown biological process",
  "gene_symbol": "POLR1C"
}